{
  "gene_name": "Cytokine-dependent hematopoietic cell linker",
  "gene_symbol": "CLNK",
  "gene": "UniProtKB:Q7Z7G1",
  "term_id": "GO:0035556",
  "term_label": "intracellular signal transduction"
}